{
  "gene": "UniProtKB:Q5ZPR3",
  "gene_symbol": "CD276",
  "term_id": "GO:0009897",
  "term_label": "external side of plasma membrane",
  "gene_name": "CD276 antigen"
}